{
  "gene_symbol": "AGAP2",
  "term_id": "GO:0003924",
  "gene": "UniProtKB:Q99490",
  "term_label": "GTPase activity",
  "gene_name": "Arf-GAP with GTPase, ANK repeat and PH domain-containing protein 2"
}